{
  "term_id": "GO:0019430",
  "gene_name": "Superoxide dismutase [Cu-Zn]",
  "term_label": "removal of superoxide radicals",
  "gene_symbol": "SOD1",
  "gene": "UniProtKB:P00441"
}